{
  "gene_symbol": "FAM166C",
  "term_label": "Unknown biological process",
  "gene_name": "Protein FAM166C",
  "term_id": "UNKNOWN:0002",
  "gene": "UniProtKB:A6NJV1"
}